repair of mitotic kinetochore microtubule attachment defect [GO:0140273] (biological process) Subtypes: positive regulation of mitotic sister chromatid biorientation [GO:0140429] Definition: The mitotic cell cycle process where kinetochore microtubule attachment defects are corrected. Relationships: is a type of repair of kinetochore microtubule attachment defect [GO:0140274]; is a type of mitotic cell cycle process [GO:1903047]; is part of GO:0007080 Also known as: correction of mitotic kinetochore microtubule attachment defects, repair of mitotic kinetochore microtubule attachment defects References: PMID:15525536